methylated-DNA-[protein]-cysteine S-methyltransferase activity [GO:0003908] (molecular function) Definition: Catalysis of the reaction: DNA (containing 6-O-methylguanine) + (protein)-L-cysteine = DNA (without 6-O-methylguanine) + protein S-methyl-L-cysteine. Relationships: is a type of S-methyltransferase activity [GO:0008172]; is a type of protein methyltransferase activity [GO:0008276] Sources: EC:2.1.1.63 Also known as: O6-alkylguanine-DNA alkyltransferase, DNA-6-O-methylguanine:[protein]-L-cysteine S-methyltransferase activity, MGMT, 6-O-methylguanine-DNA methyltransferase activity, DNA-6-O-methylguanine:protein-L-cysteine S-methyltransferase activity, O-6-methylguanine-DNA-alkyltransferase activity, methylated-DNA-protein-cysteine S-methyltransferase activity